{
  "gene_symbol": "ZNF335",
  "term_id": "GO:0006355",
  "gene_name": "Zinc finger protein 335",
  "term_label": "regulation of DNA-templated transcription",
  "gene": "UniProtKB:Q9H4Z2"
}